{
  "term_label": "Unknown molecular function",
  "gene_symbol": "FAM241B",
  "term_id": "UNKNOWN:0001",
  "gene_name": "Protein FAM241B",
  "gene": "UniProtKB:Q96D05"
}